{
  "term_id": "UNKNOWN:0001",
  "term_label": "Unknown molecular function",
  "gene_name": "Uncharacterized protein MIR1-1HG",
  "gene": "UniProtKB:Q9H1L0",
  "gene_symbol": "MIR1-1HG"
}